{
  "term_label": "intracellular protein localization",
  "gene_symbol": "SEPTIN4",
  "gene": "UniProtKB:O43236",
  "gene_name": "Septin-4",
  "term_id": "GO:0008104"
}